{
  "gene_symbol": "TUBA8",
  "term_label": "GTP binding",
  "gene_name": "Tubulin alpha-8 chain",
  "term_id": "GO:0005525",
  "gene": "UniProtKB:Q9NY65"
}